{
  "gene_symbol": "DONSON",
  "term_label": "nuclear DNA replication",
  "term_id": "GO:0033260",
  "gene_name": "Protein downstream neighbor of Son",
  "gene": "UniProtKB:Q9NYP3"
}